guanine nucleotide transmembrane transporter activity [GO:0001409] (molecular function) Definition: Enables the transfer of guanine nucleotides (GMP, GDP, and GTP) from one side of a membrane to the other. Sources: GOC:mcc Subtypes: GTP:GDP antiporter activity [GO:0010292], cyclic-GMP-AMP transmembrane transporter activity [GO:0140360], cyclic-di-GMP transmembrane transporter activity [GO:0140927], ABC-type 3',5'-cyclic GMP transmembrane transporter activity [GO:1905948] Relationships: is a type of purine nucleotide transmembrane transporter activity [GO:0015216]; is part of GO:1903790